{
  "gene_symbol": "KCND2",
  "gene_name": "Potassium voltage-gated channel subfamily D member 2",
  "gene": "UniProtKB:Q9NZV8",
  "term_id": "GO:0045211",
  "term_label": "postsynaptic membrane"
}